{
  "term_label": "plasma membrane",
  "term_id": "GO:0005886",
  "gene_name": "Olfactory receptor 1E1",
  "gene": "UniProtKB:P30953",
  "gene_symbol": "OR1E1"
}